dATP metabolic process [GO:0046060] (biological process) Definition: The chemical reactions and pathways involving dATP, deoxyadenosine triphosphate (2'-deoxyadenosine 5'-triphosphate). Sources: GOC:go_curators Also known as: dATP metabolism Relationships: is a type of GO:0009151; is a type of GO:0009215 Subtypes: dATP biosynthetic process [GO:0006175], dATP catabolic process [GO:0046061]